response to linoleic acid [GO:0070543] (biological process) Subtypes: cellular response to linoleic acid [GO:0071399] Sources: GOC:lp Relationships: is a type of response to fatty acid [GO:0070542] Also known as: response to linoleate Definition: Any process that results in a change in state or activity of a cell or an organism (in terms of movement, secretion, enzyme production, gene expression, etc.) as a result of a linoleic acid stimulus.